{
  "term_id": "GO:0004930",
  "term_label": "G protein-coupled receptor activity",
  "gene": "UniProtKB:O94910",
  "gene_name": "Adhesion G protein-coupled receptor L1",
  "gene_symbol": "ADGRL1"
}